{
  "term_id": "GO:0051642",
  "gene_symbol": "NDEL1",
  "term_label": "centrosome localization",
  "gene_name": "Nuclear distribution protein nudE-like 1",
  "gene": "UniProtKB:Q9GZM8"
}